{
  "gene_name": "Ubiquitin carboxyl-terminal hydrolase 31",
  "term_label": "Unknown molecular function",
  "gene_symbol": "USP31",
  "gene": "UniProtKB:Q70CQ4",
  "term_id": "UNKNOWN:0001"
}